D-arabinono-1,4-lactone oxidase activity [GO:0003885] (molecular function) Relationships: is a type of GO:0016899 Definition: Catalysis of the reaction: D-arabinono-1,4-lactone + O2 = dehydro-D-arabinono-1,4-lactone + H2O2 + H+. Also known as: D-arabinono-1,4-lactone:oxygen oxidoreductase activity Sources: EC:1.1.3.37, RHEA:23756